lignin catabolic process [GO:0046274] (biological process) Sources: GOC:ai Subtypes: p-hydroxyphenyl lignin catabolic process [GO:1901059], GO:1901062, syringal lignin catabolic process [GO:1901065], anaerobic lignin catabolic process [GO:1990487] Definition: The chemical reactions and pathways resulting in the breakdown of lignins, a class of polymers of phenylpropanoid units. Also known as: lignin breakdown, lignin catabolism, lignin degradation Relationships: is_a lignin metabolic process [GO:0009808]; is_a GO:0046271